arteriole smooth muscle contraction [GO:0014830] (BP) Definition: A process in which force is generated within smooth muscle tissue, resulting in a change in muscle geometry. This process occurs in the arteriole. Force generation involves a chemo-mechanical energy conversion step that is carried out by the actin/myosin complex activity, which generates force through ATP hydrolysis. The arteriole is the smallest division of the artery located between the muscular arteries and the capillaries. Sources: GOC:mtg_muscle, MA:0000706, MSH:D001160 Relationships: is a type of artery smooth muscle contraction [GO:0014824]